{
  "term_label": "L-arginine biosynthetic process",
  "gene": "UniProtKB:Q8N159",
  "term_id": "GO:0006526",
  "gene_name": "N-acetylglutamate synthase, mitochondrial",
  "gene_symbol": "NAGS"
}